{
  "term_label": "cytoplasm",
  "gene_name": "Phosphatidylinositol 3-kinase catalytic subunit type 3",
  "gene_symbol": "PIK3C3",
  "gene": "UniProtKB:Q8NEB9",
  "term_id": "GO:0005737"
}